{
  "gene_symbol": "RNASEH2A",
  "term_id": "GO:0006298",
  "gene": "UniProtKB:O75792",
  "gene_name": "Ribonuclease H2 subunit A",
  "term_label": "mismatch repair"
}